{
  "gene_symbol": "MSTO1",
  "term_label": "mitochondrion",
  "gene": "UniProtKB:Q9BUK6",
  "gene_name": "Protein misato homolog 1",
  "term_id": "GO:0005739"
}